{
  "gene_name": "Heat shock 70 kDa protein 13",
  "gene_symbol": "HSPA13",
  "term_label": "cytosol",
  "gene": "UniProtKB:P48723",
  "term_id": "GO:0005829"
}